{
  "gene_name": "Mucin-15",
  "term_id": "UNKNOWN:0002",
  "gene": "UniProtKB:Q8N387",
  "term_label": "Unknown biological process",
  "gene_symbol": "MUC15"
}